{
  "term_id": "GO:0005768",
  "term_label": "endosome",
  "gene": "UniProtKB:Q6IQ22",
  "gene_name": "Ras-related protein Rab-12",
  "gene_symbol": "RAB12"
}